organelle envelope lumen [GO:0031970] (cellular component) Relationships: is_a intracellular organelle lumen [GO:0070013]; is part of organelle envelope [GO:0031967] Sources: GOC:mah Definition: The region between the inner and outer lipid bilayers of an organelle envelope. Also known as: organelle intermembrane space Subtypes: nuclear envelope lumen [GO:0005641], mitochondrial intermembrane space [GO:0005758], plastid intermembrane space [GO:0009529]